{
  "gene_name": "Pituitary adenylate cyclase-activating polypeptide",
  "gene_symbol": "ADCYAP1",
  "term_label": "positive regulation of cAMP/PKA signal transduction",
  "term_id": "GO:0141163",
  "gene": "UniProtKB:P18509"
}